{
  "term_id": "UNKNOWN:0002",
  "gene_symbol": "SMCR5",
  "gene": "UniProtKB:Q8TEV8",
  "term_label": "Unknown biological process",
  "gene_name": "Smith-Magenis syndrome chromosomal region candidate gene 5 protein"
}